{
  "gene_symbol": "PCNA",
  "term_label": "translesion synthesis",
  "gene": "UniProtKB:P12004",
  "gene_name": "Proliferating cell nuclear antigen",
  "term_id": "GO:0019985"
}